{
  "gene": "UniProtKB:A6PVC2",
  "gene_name": "Protein monoglycylase TTLL8",
  "term_label": "flagellated sperm motility",
  "gene_symbol": "TTLL8",
  "term_id": "GO:0030317"
}